inositol trisphosphate phosphatase activity [GO:0046030] (molecular function) Relationships: is a type of inositol phosphate phosphatase activity [GO:0052745] Sources: GOC:bf Definition: Catalysis of the reaction: myo-inositol trisphosphate + H2O = myo-inositol bisphosphate + phosphate. Also known as: IP(3) phosphatase activity, IP3 phosphatase activity Subtypes: inositol-polyphosphate 5-phosphatase activity [GO:0004445], GO:0017161, inositol-1,3,4-trisphosphate 1-phosphatase activity [GO:0052829], GO:1990640, inositol-4,5,6-triphosphate 5-phosphatase activity [GO:1990648]